{
  "gene_symbol": "SALL1",
  "gene_name": "Sal-like protein 1",
  "term_id": "GO:0005634",
  "term_label": "nucleus",
  "gene": "UniProtKB:Q9NSC2"
}